{
  "term_label": "Unknown cellular component",
  "gene_symbol": "KRTAP4-9",
  "gene": "UniProtKB:Q9BYQ8",
  "term_id": "UNKNOWN:0003",
  "gene_name": "Keratin-associated protein 4-9"
}